{
  "term_label": "ciliary transition zone",
  "term_id": "GO:0035869",
  "gene_symbol": "CIBAR1",
  "gene": "UniProtKB:A1XBS5",
  "gene_name": "CBY1-interacting BAR domain-containing protein 1"
}